phospholipid scramblase activity [GO:0017128] (molecular function) Definition: Catalysis of the movement of phospholipids from one membrane bilayer leaflet to the other, by an ATP-independent mechanism. Note: Nomenclature note. Scramblases are ATP-independent, non-selective, translocases inducing non-specific transbilayer movements across the membrane. Flippases and floppases are ATP-dependent transbilayer lipid translocators. According to an extensively used, though not universal, nomenclature, they catalyze lipid transfer towards the inward monolayer (flippases) or towards the outward monolayer (floppases). Relationships: is a type of phospholipid transporter activity [GO:0005548]; is a type of intramembrane lipid transporter activity [GO:0140303]; BFO_0000050 GO:0017121 References: PMID:20043909, PMID:20302864 Sources: GOC:cjm Regulation: positively regulated by positive regulation of phospholipid scramblase activity [GO:1900163]